{
  "gene": "UniProtKB:Q9Y4P3",
  "term_label": "endoplasmic reticulum",
  "gene_symbol": "TBL2",
  "term_id": "GO:0005783",
  "gene_name": "Transducin beta-like protein 2"
}